L-leucine catabolic process [GO:0006552] (BP) Sources: GOC:ai Relationships: is a type of L-leucine metabolic process [GO:0006551]; is a type of branched-chain amino acid catabolic process [GO:0009083]; is a type of L-amino acid catabolic process [GO:0170035]; is a type of proteinogenic amino acid catabolic process [GO:0170040] Definition: The chemical reactions and pathways resulting in the breakdown of L-leucine, 2-amino-4-methylpentanoic acid. Also known as: leucine catabolic process, L-leucine breakdown, L-leucine catabolism, L-leucine degradation